ribosomal subunit [GO:0044391] (cellular component) Relationships: is a type of ribonucleoprotein complex [GO:1990904]; is part of ribosome [GO:0005840] Definition: Either of the two subunits of a ribosome: the ribosomal large subunit or the ribosomal small subunit. Subtypes: large ribosomal subunit [GO:0015934], small ribosomal subunit [GO:0015935] Sources: GOC:jl